{
  "gene": "UniProtKB:O75071",
  "gene_symbol": "EFCAB14",
  "gene_name": "EF-hand calcium-binding domain-containing protein 14",
  "term_label": "Unknown biological process",
  "term_id": "UNKNOWN:0002"
}